{
  "gene_name": "Dexamethasone-induced Ras-related protein 1",
  "term_id": "GO:0007165",
  "gene": "UniProtKB:Q9Y272",
  "term_label": "signal transduction",
  "gene_symbol": "RASD1"
}